shikimate transmembrane transport [GO:0015733] (biological process) Definition: The process in which shikimate is transported across a lipid bilayer, from one side of a membrane to the other. Sources: GOC:krc Also known as: shikimate transport Relationships: is a type of monocarboxylic acid transport [GO:0015718]; is a type of organic hydroxy compound transport [GO:0015850]; is_a GO:1905039